cytosolic lipolysis [GO:0061725] (biological process) Definition: The chemical reactions and pathways resulting in the breakdown of lipid droplets and hydrolysis of stored triglycerides occurring through the orchestrated activation of cytosolic lipases. Sources: GOC:autophagy Relationships: is_a lipid catabolic process [GO:0016042]; occurs in cytosol [GO:0005829]